{
  "term_label": "protein import into nucleus",
  "gene_symbol": "NUP107",
  "gene": "UniProtKB:P57740",
  "term_id": "GO:0006606",
  "gene_name": "Nuclear pore complex protein Nup107"
}